{
  "gene": "UniProtKB:O75486",
  "gene_name": "Transcription initiation protein SPT3 homolog",
  "term_id": "UNKNOWN:0002",
  "gene_symbol": "SUPT3H",
  "term_label": "Unknown biological process"
}